{
  "gene_name": "E3 ubiquitin-protein ligase RAD18",
  "gene": "UniProtKB:Q9NS91",
  "term_id": "GO:0006301",
  "gene_symbol": "RAD18",
  "term_label": "DNA damage tolerance"
}